{
  "term_label": "Unknown molecular function",
  "gene_name": "Cilia- and flagella-associated protein 52",
  "gene": "UniProtKB:Q8N1V2",
  "term_id": "UNKNOWN:0001",
  "gene_symbol": "CFAP52"
}